{
  "gene": "UniProtKB:Q3ZLR7",
  "gene_symbol": "SUPT20HL1",
  "gene_name": "Transcription factor SPT20 homolog-like 1",
  "term_id": "GO:0000124",
  "term_label": "SAGA complex"
}